{
  "gene": "UniProtKB:Q07869",
  "term_label": "intracellular receptor signaling pathway",
  "gene_symbol": "PPARA",
  "term_id": "GO:0030522",
  "gene_name": "Peroxisome proliferator-activated receptor alpha"
}